{
  "gene": "UniProtKB:B4E2M5",
  "gene_symbol": "ANKRD66",
  "term_id": "UNKNOWN:0001",
  "term_label": "Unknown molecular function",
  "gene_name": "Ankyrin repeat domain-containing protein 66"
}